{
  "term_id": "UNKNOWN:0002",
  "term_label": "Unknown biological process",
  "gene_symbol": "CYB5R2",
  "gene_name": "NADH-cytochrome b5 reductase 2",
  "gene": "UniProtKB:Q6BCY4"
}